{
  "term_id": "GO:0005795",
  "gene_name": "Alpha-1,3-mannosyl-glycoprotein 4-beta-N-acetylglucosaminyltransferase-like protein MGAT4D",
  "term_label": "Golgi stack",
  "gene": "UniProtKB:A6NG13",
  "gene_symbol": "MGAT4D"
}